peptide hormone secretion [GO:0030072] (biological process) Relationships: is a type of peptide secretion [GO:0002790]; is a type of hormone secretion [GO:0046879] Sources: GOC:mah Subtypes: insulin secretion [GO:0030073], vasopressin secretion [GO:0030103], GO:0030252, melanocyte-stimulating hormone secretion [GO:0036160], GO:0036161, GO:0036321, pancreatic polypeptide secretion [GO:0036322], corticotropin-releasing hormone secretion [GO:0043396], GO:0051458, GO:0070091, somatostatin secretion [GO:0070253], prolactin secretion [GO:0070459], GO:0070460, mating pheromone secretion [GO:0071834], peptide pheromone secretion [GO:0090538], substance P secretion [GO:1990772] Definition: The regulated release of a peptide hormone from a cell. Regulation: RO_0002211 by regulation of peptide hormone secretion [GO:0090276]; positively regulated by positive regulation of peptide hormone secretion [GO:0090277]; negatively regulated by negative regulation of peptide hormone secretion [GO:0090278]